{
  "gene_name": "Spermatogenesis-associated protein 12",
  "term_label": "Unknown cellular component",
  "term_id": "UNKNOWN:0003",
  "gene": "UniProtKB:Q7Z6I5",
  "gene_symbol": "SPATA12"
}